{
  "term_label": "synapse",
  "gene_name": "Cerebellin-3",
  "gene_symbol": "CBLN3",
  "term_id": "GO:0045202",
  "gene": "UniProtKB:Q6UW01"
}